{
  "gene": "UniProtKB:Q96EH8",
  "term_id": "GO:0005769",
  "gene_name": "E3 ubiquitin-protein ligase NEURL3",
  "gene_symbol": "NEURL3",
  "term_label": "early endosome"
}